{
  "gene_name": "Immunoglobulin lambda joining 6 (Fragment)",
  "term_id": "UNKNOWN:0001",
  "gene": "UniProtKB:A0A0A0MT93",
  "term_label": "Unknown molecular function",
  "gene_symbol": "IGLJ6"
}